{
  "gene": "UniProtKB:Q04206",
  "gene_name": "Transcription factor p65",
  "term_label": "DNA-binding transcription factor activity, RNA polymerase II-specific",
  "term_id": "GO:0000981",
  "gene_symbol": "RELA"
}